taurine dioxygenase activity [GO:0000908] (molecular function) Also known as: 2-aminoethanesulfonate dioxygenase activity, alpha-ketoglutarate-dependent taurine dioxygenase activity, taurine, 2-oxoglutarate:O2 oxidoreductase (sulfite-forming) Sources: EC:1.14.11.17, RHEA:15909 Definition: Catalysis of the reaction: 2-oxoglutarate + O2 + taurine = aminoacetaldehyde + CO2 + succinate + sulfite. Relationships: is a type of GO:0016706